copper import into the mitochondrion [GO:0140636] (BP) Relationships: is a type of copper ion transmembrane transport [GO:0035434] References: PMID:32979421 Definition: The process in which copper is transported from the cytosol into the mitochondrial matrix.